rhamnolipid biosynthesis [GO:0106236] (biological process) Also known as: rhamnolipid production Relationships: is a type of glycolipid biosynthetic process [GO:0009247] Definition: The chemical reactions and pathways resulting in the formation/production of a glycolipid surfactant that acts as a bacterial biofilm dispersal. References: PMID:28715477 Sources: GOC:vw